kinase activity [GO:0016301] (MF) Sources: ISBN:0198506732 Also known as: phosphokinase activity Relationships: is a type of transferase activity, transferring phosphorus-containing groups [GO:0016772] Note: Note that this term encompasses all activities that transfer a single phosphate group; although ATP is by far the most common phosphate donor, reactions using other phosphate donors are included in this term. Regulation: regulated by GO:0019207; positively regulated by kinase activator activity [GO:0019209]; negatively regulated by kinase inhibitor activity [GO:0019210]; RO_0002212 by GO:0033673; positively regulated by positive regulation of kinase activity [GO:0033674]; regulated by regulation of kinase activity [GO:0043549] Subtypes: lipid kinase activity [GO:0001727], NAD+ kinase activity [GO:0003951], acetylglutamate kinase activity [GO:0003991], adenylylsulfate kinase activity [GO:0004020], choline kinase activity [GO:0004103], creatine kinase activity [GO:0004111], dephospho-CoA kinase activity [GO:0004140], dolichol kinase activity [GO:0004168], ethanolamine kinase activity [GO:0004305], glycerol kinase activity [GO:0004370], glycerone kinase activity [GO:0004371], hydroxyethylthiazole kinase activity [GO:0004417], mevalonate kinase activity [GO:0004496], GO:0004594, phosphoglycerate kinase activity [GO:0004618], phosphomevalonate kinase activity [GO:0004631], protein kinase activity [GO:0004672], selenide, water dikinase activity [GO:0004756], shikimate kinase activity [GO:0004765], pyridoxal kinase activity [GO:0008478], riboflavin kinase activity [GO:0008531], GO:0008776, carbamate kinase activity [GO:0008804], glycerate kinase activity [GO:0008887], hydroxymethylpyrimidine kinase activity [GO:0008902], inosine kinase activity [GO:0008906], phosphomethylpyrimidine kinase activity [GO:0008972], phosphoribulokinase activity [GO:0008974], polyphosphate kinase activity [GO:0008976], GO:0008980, GO:0008986, tagatose-6-phosphate kinase activity [GO:0009024], lipid-A 4'-kinase activity [GO:0009029], thiamine-phosphate kinase activity [GO:0009030], undecaprenol kinase activity [GO:0009038], phytol kinase activity [GO:0010276], phenol kinase activity [GO:0018720], inositol 3-kinase activity [GO:0019140], thiamine kinase activity [GO:0019165], GO:0019200, GO:0019202, nucleobase-containing compound kinase activity [GO:0019205], aminoglycoside phosphotransferase activity [GO:0034071], NADH kinase activity [GO:0042736], adenosylcobinamide kinase activity [GO:0043752], glycerate 2-kinase activity [GO:0043798], ADP-specific glucokinase activity [GO:0043843], ADP-specific phosphofructokinase activity [GO:0043844], L-seryl-tRNA(Sec) kinase activity [GO:0043915], gluconokinase activity [GO:0046316], S-methyl-5-thioribose kinase activity [GO:0046522], GO:0047321, phosphoenolpyruvate-glycerone phosphotransferase activity [GO:0047324], glycerol-3-phosphate-glucose phosphotransferase activity [GO:0047327], acyl-phosphate-hexose phosphotransferase activity [GO:0047328], phosphoramidate-hexose phosphotransferase activity [GO:0047329], polyphosphate-glucose phosphotransferase activity [GO:0047330], diphosphate-glycerol phosphotransferase activity [GO:0047331], diphosphate-serine phosphotransferase activity [GO:0047332], 5-methyldeoxycytidine-5'-phosphate kinase activity [GO:0047336], 5-dehydro-2-deoxygluconokinase activity [GO:0047590], acetate kinase (diphosphate) activity [GO:0047601], GO:0047620, ADP-thymidine kinase activity [GO:0047628], GO:0047633, GO:0047649, alkylglycerone kinase activity [GO:0047650], GO:0047666, AMP-thymidine kinase activity [GO:0047667], beta-glucoside kinase activity [GO:0047700], GO:0047715, ATP:2-methylpropanoate phosphotransferase activity [GO:0047758], GO:0047761, D-arabinokinase activity [GO:0047814], GO:0047841, erythritol kinase activity [GO:0047878], GO:0047887, GO:0047900, galacturonokinase activity [GO:0047912], glucosamine kinase activity [GO:0047931], glucose-1,6-bisphosphate synthase activity [GO:0047933], glucose-1-phosphate phosphodismutase activity [GO:0047937], glucuronokinase activity [GO:0047940], guanidinoacetate kinase activity [GO:0047973], GO:0047976, GO:0050059, GO:0050073, opheline kinase activity [GO:0050154], GO:0050165, phosphoglucokinase activity [GO:0050190], GO:0050191, phosphoribokinase activity [GO:0050195], fucokinase activity [GO:0050201], GO:0050225, riboflavin phosphotransferase activity [GO:0050257], ribosylnicotinamide kinase activity [GO:0050262], GO:0050276, sedoheptulokinase activity [GO:0050277], tagatose kinase activity [GO:0050317], taurocyamine kinase activity [GO:0050324], thiamine-diphosphate kinase activity [GO:0050331], triokinase activity [GO:0050354], viomycin kinase activity [GO:0050394], xylitol kinase activity [GO:0050400], 4-(cytidine 5'-diphospho)-2-C-methyl-D-erythritol kinase activity [GO:0050515], alpha-glucan, water dikinase activity [GO:0050521], phosphoglucan, water dikinase activity [GO:0051752], nicotinate riboside kinase activity [GO:0061769], autoinducer-2 kinase activity [GO:0071518], GO:0102194, ecdysteroid 22-kinase activity [GO:0106389], 4-hydroxytryptamine kinase activity [GO:0140383], muramyl dipeptide kinase activity [GO:0160047], inositol phosphate kinase activity [GO:0180030] Definition: Catalysis of the transfer of a phosphate group, usually from ATP, to a substrate molecule.